{
  "gene": "UniProtKB:Q9Y5G4",
  "term_label": "cell adhesion",
  "gene_name": "Protocadherin gamma-A9",
  "gene_symbol": "PCDHGA9",
  "term_id": "GO:0007155"
}